{
  "term_label": "DNA-binding transcription factor activity, RNA polymerase II-specific",
  "gene": "UniProtKB:Q8TD17",
  "term_id": "GO:0000981",
  "gene_name": "Zinc finger protein 398",
  "gene_symbol": "ZNF398"
}